{
  "gene_symbol": "FOCAD",
  "term_id": "UNKNOWN:0001",
  "gene_name": "Focadhesin",
  "gene": "UniProtKB:Q5VW36",
  "term_label": "Unknown molecular function"
}